nuclear mRNA surveillance of meiosis-specific transcripts [GO:0033621] (biological process) Definition: The chemical reactions and pathways resulting in the selective degradation of meiosis-specific transcripts during vegetative growth, by a mechanism that requires determinant of selective removal (DSR) sequences in the targeted mRNAs and involves a YTH family protein. Regulation: RO_0002211 by GO:0120270; negatively regulated by GO:0120271; positively regulated by positive regulation of nuclear mRNA surveillance of meiosis-specific transcripts [GO:0120272] References: PMID:16823445 Also known as: degradation of meiosis-specific transcripts, mRNA breakdown, meiosis-specific transcripts, mRNA catabolism, meiosis-specific transcripts, mRNA degradation, meiosis-specific transcripts, nuclear mRNA catabolic process, meiosis-specific transcripts, nuclear-transcribed mRNA catabolic process, meiosis-specific transcripts Relationships: is a type of nuclear mRNA surveillance [GO:0071028] Note: Note that it is speculated that higher eukaryotic YTH-family protein may be involved in similar mechanisms to suppress gene regulation during gametogenesis or general silencing.